recombination hotspot binding [GO:0010844] (molecular function) Definition: Binding to a genomic region which promotes recombination. Sources: GOC:dph, GOC:tb Also known as: DNA binding, recombination hotspot Relationships: is a type of DNA binding [GO:0003677]